{
  "gene_name": "Type-2 angiotensin II receptor",
  "term_id": "GO:0004945",
  "gene_symbol": "AGTR2",
  "gene": "UniProtKB:P50052",
  "term_label": "angiotensin type II receptor activity"
}